{
  "term_label": "sensory perception of smell",
  "gene": "UniProtKB:Q8NGQ6",
  "term_id": "GO:0007608",
  "gene_symbol": "OR9I1",
  "gene_name": "Olfactory receptor 9I1"
}